nuclear membrane protein complex [GO:0106083] (cellular component) Subtypes: GO:0106094 Relationships: is a type of membrane protein complex [GO:0098796]; is a type of GO:0140513; is part of nuclear envelope [GO:0005635] Definition: Any protein complex that is part of the nuclear membrane. References: PMID:28356353 Sources: GOC:lnp